regulation of ferulate catabolic process [GO:1901466] (biological process) Definition: Any process that modulates the frequency, rate or extent of ferulate catabolic process. Sources: GOC:TermGenie, GOC:mengo_curators Also known as: regulation of ferulate breakdown, regulation of ferulate catabolism, regulation of ferulate degradation Relationships: is a type of regulation of catabolic process [GO:0009894]; is a type of regulation of ketone metabolic process [GO:0010565]; is a type of regulation of small molecule metabolic process [GO:0062012]; regulates ferulate catabolic process [GO:1901067] Subtypes: negative regulation of ferulate catabolic process [GO:1901467], positive regulation of ferulate catabolic process [GO:1901468]